{
  "term_label": "DNA-binding transcription factor activity, RNA polymerase II-specific",
  "gene_symbol": "NRL",
  "gene": "UniProtKB:P54845",
  "gene_name": "Neural retina-specific leucine zipper protein",
  "term_id": "GO:0000981"
}